cystoblast division [GO:0007282] (biological process) Definition: Any of the rounds of incomplete mitosis undergone by a cystoblast to form a cyst of interconnected cells. References: PMID:21452446 Also known as: cystoblast cell division Relationships: is a type of asymmetric cell division [GO:0008356]; is part of germ cell development [GO:0007281] Subtypes: germarium-derived cystoblast division [GO:0048142]